{
  "gene": "UniProtKB:Q8IWA0",
  "term_id": "GO:0005730",
  "gene_symbol": "WDR75",
  "gene_name": "WD repeat-containing protein 75",
  "term_label": "nucleolus"
}